{
  "term_id": "GO:0032511",
  "term_label": "late endosome to vacuole transport via multivesicular body sorting pathway",
  "gene": "UniProtKB:Q9H444",
  "gene_name": "Charged multivesicular body protein 4b",
  "gene_symbol": "CHMP4B"
}